{
  "gene_symbol": "SWAP70",
  "term_id": "UNKNOWN:0001",
  "term_label": "Unknown molecular function",
  "gene": "UniProtKB:Q9UH65",
  "gene_name": "Switch-associated protein 70"
}